{
  "gene_name": "C-C chemokine receptor-like 2",
  "term_id": "GO:0006955",
  "term_label": "immune response",
  "gene": "UniProtKB:O00421",
  "gene_symbol": "CCRL2"
}